contractile actin filament bundle [GO:0097517] (cellular component) Sources: GOC:cjm, GOC:mah, ISBN:0815316194 Definition: An actin filament bundle in which the filaments are loosely packed (approximately 30-60 nm apart) and arranged with opposing polarities; the loose packing allows myosin (usually myosin-II) to enter the bundle. Subtypes: stress fiber [GO:0001725] Relationships: is a type of actin filament bundle [GO:0032432]